{
  "gene_name": "Complement receptor type 1",
  "gene_symbol": "CR1",
  "term_id": "GO:0005886",
  "term_label": "plasma membrane",
  "gene": "UniProtKB:P17927"
}